high-affinity IgE receptor activity [GO:0019768] (molecular function) Definition: Combining with high affinity with an immunoglobulin of the IgE isotype via the Fc region, and transmitting the signal from one side of the membrane to the other to initiate a change in cell activity. Also known as: high affinity IgE receptor activity, high affinity Fc receptor activity Relationships: is a type of IgE receptor activity [GO:0019767] Sources: GOC:add, GOC:signaling, ISBN:0781735149